cellular response to differentiation-inducing factor 2 [GO:0061862] (biological process) Also known as: cellular response to 1-(3,5-dichloro-2,6-dihydroxy-4-methoxyphenyl)pentan-1-one, cellular response to DIF-2, cellular response to DIF2 Relationships: is a type of cellular response to stimulus [GO:0051716]; is a type of response to differentiation-inducing factor 2 [GO:1905960] References: PMID:19684855 Definition: Any process that results in a change in state or activity of a cell (in terms of movement, secretion, enzyme production, gene expression, etc.) as a result of a 1-(3,5-dichloro-2,6-dihydroxy-4-methoxyphenyl)pentan-1-one stimulus.